positive regulation of interleukin-18 production [GO:0032741] (biological process) Definition: Any process that activates or increases the frequency, rate, or extent of interleukin-18 production. Sources: GOC:mah Also known as: positive regulation of IL-18 production, up regulation of interleukin-18 production, up-regulation of interleukin-18 production, upregulation of interleukin-18 production, activation of interleukin-18 production, positive regulation of interleukin-18 biosynthetic process, positive regulation of interleukin-18 secretion, stimulation of interleukin-18 production Relationships: is a type of GO:0001819; is a type of regulation of interleukin-18 production [GO:0032661]; positively regulates interleukin-18 production [GO:0032621]